{
  "gene_symbol": "LHX6",
  "gene": "UniProtKB:Q9UPM6",
  "gene_name": "LIM_homeobox protein Lhx6",
  "term_id": "GO:0021884",
  "term_label": "forebrain neuron development"
}